{
  "gene_symbol": "RNASEH2C",
  "term_label": "ribonuclease H2 complex",
  "gene_name": "Ribonuclease H2 subunit C",
  "gene": "UniProtKB:Q8TDP1",
  "term_id": "GO:0032299"
}